positive regulation of locomotion involved in locomotory behavior [GO:0090326] (biological process) Sources: GOC:dph, GOC:kmv, GOC:tb Definition: Any process that increases the frequency, rate, or extent of the self-propelled movement of a cell or organism from one location to another in a behavioral context; the aspect of locomotory behavior having to do with movement. Relationships: is a type of positive regulation of locomotion [GO:0040017]; is_a positive regulation of behavior [GO:0048520]; is a type of regulation of locomotion involved in locomotory behavior [GO:0090325]; positively regulates locomotion involved in locomotory behavior [GO:0031987]